dolichyl-diphosphate-polyphosphate phosphotransferase activity [GO:0047337] (molecular function) Definition: Catalysis of the reaction: dolichyl diphosphate + long-chain-polyphosphate = dolichol-phosphate + long-chain-polyphosphate. Sources: EC:2.7.4.20, MetaCyc:2.7.4.20-RXN Also known as: dolichyl-diphosphate:polyphosphate phosphotransferase activity, dolichylpyrophosphate:polyphosphate phosphotransferase activity Relationships: is a type of phosphotransferase activity, phosphate group as acceptor [GO:0016776]